{
  "term_id": "GO:0005794",
  "term_label": "Golgi apparatus",
  "gene": "UniProtKB:O75711",
  "gene_name": "Scrapie-responsive protein 1",
  "gene_symbol": "SCRG1"
}